{
  "gene": "UniProtKB:P22087",
  "gene_name": "rRNA 2'-O-methyltransferase fibrillarin",
  "term_label": "rRNA methylation",
  "gene_symbol": "FBL",
  "term_id": "GO:0031167"
}